{
  "gene": "UniProtKB:Q9Y5Y0",
  "term_id": "GO:0016020",
  "gene_symbol": "FLVCR1",
  "gene_name": "Heme transporter FLVCR1",
  "term_label": "membrane"
}